{
  "gene_name": "Zinc finger protein 518B",
  "term_id": "GO:0000981",
  "term_label": "DNA-binding transcription factor activity, RNA polymerase II-specific",
  "gene": "UniProtKB:Q9C0D4",
  "gene_symbol": "ZNF518B"
}